{
  "term_id": "GO:0005886",
  "term_label": "plasma membrane",
  "gene": "UniProtKB:Q8NGU9",
  "gene_name": "Probable G-protein coupled receptor 150",
  "gene_symbol": "GPR150"
}